{
  "gene": "UniProtKB:O43670",
  "term_label": "spindle matrix",
  "gene_symbol": "ZNF207",
  "gene_name": "BUB3-interacting and GLEBS motif-containing protein ZNF207",
  "term_id": "GO:1990047"
}